blastocyst growth [GO:0001832] (biological process) Definition: An increase in size of a blastocyst due to expansion of the blastocoelic cavity cell shape changes and cell proliferation. Sources: GOC:dph, ISBN:0124020607, ISBN:0198542771 Note: See also the Anatomical Dictionary for Mouse Development ontology terms 'TS4, blastocoelic cavity ; EMAP:17', 'TS5, blastocoelic cavity ; EMAP:27' and 'TS6, blastocoelic cavity ; EMAP:36'. Relationships: is a type of GO:0048589; is part of blastocyst development [GO:0001824] Also known as: blastula growth